sesquiterpenoid catabolic process [GO:0016107] (biological process) Definition: The chemical reactions and pathways resulting in the breakdown of sesquiterpenoid compounds, terpenoids with three isoprene units. Also known as: sesquiterpenoid breakdown, sesquiterpenoid catabolism, sesquiterpenoid degradation Relationships: is a type of sesquiterpenoid metabolic process [GO:0006714]; is a type of terpenoid catabolic process [GO:0016115] Sources: GOC:go_curators Subtypes: juvenile hormone catabolic process [GO:0006719], GO:0016488, GO:0046345, pentalenolactone catabolic process [GO:1901779], GO:1901942